{
  "gene_name": "Putative tyrosine carboxypeptidase MATCAP2",
  "term_id": "UNKNOWN:0001",
  "gene_symbol": "MATCAP2",
  "term_label": "Unknown molecular function",
  "gene": "UniProtKB:Q8NCT3"
}